intracellular cholesterol transport [GO:0032367] (BP) Definition: The directed movement of cholesterol, cholest-5-en-3-beta-ol, within cells. Sources: GOC:mah Relationships: is a type of cholesterol transport [GO:0030301]; is a type of intracellular sterol transport [GO:0032366] Subtypes: vesicle-mediated cholesterol transport [GO:0090119], lysosome to ER cholesterol transport [GO:0090120] Regulation: regulated by regulation of intracellular cholesterol transport [GO:0032383]; negatively regulated by negative regulation of intracellular cholesterol transport [GO:0032384]; positively regulated by positive regulation of intracellular cholesterol transport [GO:0032385]